negative regulation of toll-like receptor 6 signaling pathway [GO:0034152] (biological process) Definition: Any process that stops, prevents, or reduces the frequency, rate, or extent of toll-like receptor 6 signaling pathway. References: PMID:16551253, PMID:17328678 Sources: GOC:add Also known as: negative regulation of TLR6 signaling pathway, negative regulation of toll-like receptor 6 signalling pathway Relationships: is a type of GO:0002683; is a type of negative regulation of signal transduction [GO:0009968]; is a type of regulation of toll-like receptor 6 signaling pathway [GO:0034151]; negatively regulates toll-like receptor 6 signaling pathway [GO:0034150]